{
  "gene_symbol": "SWAP70",
  "term_label": "nucleus",
  "gene_name": "Switch-associated protein 70",
  "term_id": "GO:0005634",
  "gene": "UniProtKB:Q9UH65"
}